endogalactosaminidase activity [GO:0033931] (molecular function) Definition: Catalysis of the endohydrolysis of (1->4)-alpha-D-galactosaminidic linkages in poly(D-galactosamine). Relationships: is a type of hexosaminidase activity [GO:0015929] Also known as: galactosaminoglycan glycanohydrolase activity Sources: EC:3.2.1.109 Subtypes: chondroitin hydrolase activity [GO:0052757]